{
  "term_id": "UNKNOWN:0002",
  "gene": "UniProtKB:O14776",
  "gene_symbol": "TCERG1",
  "gene_name": "Transcription elongation regulator 1",
  "term_label": "Unknown biological process"
}